{
  "term_id": "GO:0042147",
  "term_label": "retrograde transport, endosome to Golgi",
  "gene_name": "Ras-related protein Rab-6B",
  "gene_symbol": "RAB6B",
  "gene": "UniProtKB:Q9NRW1"
}